positive regulation of behavioral fear response [GO:2000987] (BP) Also known as: positive regulation of behavioural fear response Definition: Any process that activates or increases the frequency, rate or extent of behavioral fear response. Relationships: is a type of positive regulation of defense response [GO:0031349]; is_a positive regulation of behavior [GO:0048520]; is a type of positive regulation of fear response [GO:1903367]; is a type of regulation of behavioral fear response [GO:2000822]; positively regulates GO:0001662 Sources: GOC:obol